{
  "term_label": "interstitial matrix",
  "gene": "UniProtKB:Q6UXI7",
  "gene_symbol": "VIT",
  "gene_name": "Vitrin",
  "term_id": "GO:0005614"
}